{
  "gene_name": "RAD52 motif-containing protein 1",
  "term_label": "Unknown molecular function",
  "gene_symbol": "RDM1",
  "term_id": "UNKNOWN:0001",
  "gene": "UniProtKB:Q8NG50"
}